cardiac right atrium formation [GO:0003217] (biological process) Definition: The developmental process pertaining to the initial formation of a cardiac right atrium from unspecified parts. Sources: GOC:mtg_heart Relationships: is a type of cardiac atrium formation [GO:0003210]; is part of GO:0003213